{
  "gene_symbol": "IFNL3",
  "term_label": "innate immune response",
  "gene_name": "Interferon lambda-3",
  "term_id": "GO:0045087",
  "gene": "UniProtKB:Q8IZI9"
}